{
  "gene_name": "Protein S100-A4",
  "gene_symbol": "S100A4",
  "term_label": "extracellular space",
  "gene": "UniProtKB:P26447",
  "term_id": "GO:0005615"
}